{
  "gene_symbol": "KRTAP4-7",
  "gene": "UniProtKB:Q9BYR0",
  "term_id": "UNKNOWN:0001",
  "gene_name": "Keratin-associated protein 4-7",
  "term_label": "Unknown molecular function"
}